{
  "gene": "UniProtKB:Q11130",
  "gene_name": "Alpha-(1,3)-fucosyltransferase 7",
  "gene_symbol": "FUT7",
  "term_id": "GO:0017083",
  "term_label": "4-galactosyl-N-acetylglucosaminide 3-alpha-L-fucosyltransferase activity"
}